{
  "term_id": "GO:0000981",
  "term_label": "DNA-binding transcription factor activity, RNA polymerase II-specific",
  "gene": "UniProtKB:O43298",
  "gene_symbol": "ZBTB43",
  "gene_name": "Zinc finger and BTB domain-containing protein 43"
}